{
  "term_label": "Unknown molecular function",
  "gene": "UniProtKB:Q7Z6M4",
  "gene_name": "Transcription termination factor 4, mitochondrial",
  "gene_symbol": "MTERF4",
  "term_id": "UNKNOWN:0001"
}